vacuole fusion, non-autophagic [GO:0042144] (biological process) Sources: GOC:jl Relationships: is a type of GO:0097576 Regulation: regulated by regulation of vacuole fusion, non-autophagic [GO:0032889]; positively regulated by positive regulation of vacuole fusion, non-autophagic [GO:0061191]; negatively regulated by negative regulation of vacuole fusion, non-autophagic [GO:0061192] Also known as: homotypic vacuole fusion, homotypic vacuole fusion (non-autophagic), homotypic vacuole fusion, non-autophagic, vacuole fusion (non-autophagic) Definition: The fusion of two vacuole membranes to form a single vacuole.